tetrapyrrole binding [GO:0046906] (molecular function) Sources: GOC:curators, ISBN:0198506732 Also known as: porphyrin binding Subtypes: chlorophyll binding [GO:0016168], heme binding [GO:0020037], cobalamin binding [GO:0031419] Definition: Binding to a tetrapyrrole, a compound containing four pyrrole nuclei variously substituted and linked to each other through carbons at the alpha position. Relationships: is a type of binding [GO:0005488]